{
  "gene_name": "Transmembrane protein LOC653160",
  "gene": "UniProtKB:Q7L0L9",
  "term_id": "UNKNOWN:0002",
  "term_label": "Unknown biological process",
  "gene_symbol": "Q7L0L9"
}